{
  "gene_name": "Cell cycle checkpoint control protein RAD9A",
  "term_id": "GO:0071479",
  "gene_symbol": "RAD9A",
  "gene": "UniProtKB:Q99638",
  "term_label": "cellular response to ionizing radiation"
}